{
  "gene": "UniProtKB:Q2NKX8",
  "term_label": "Unknown cellular component",
  "term_id": "UNKNOWN:0003",
  "gene_name": "DNA excision repair protein ERCC-6-like",
  "gene_symbol": "ERCC6L"
}